{
  "gene_name": "Peroxisomal membrane protein 11B",
  "gene_symbol": "PEX11B",
  "term_label": "Unknown molecular function",
  "term_id": "UNKNOWN:0001",
  "gene": "UniProtKB:O96011"
}